{
  "term_id": "GO:0008333",
  "gene": "UniProtKB:P51809",
  "term_label": "endosome to lysosome transport",
  "gene_name": "Vesicle-associated membrane protein 7",
  "gene_symbol": "VAMP7"
}